{
  "gene": "UniProtKB:Q9UBK5",
  "term_label": "positive regulation of phosphatidylinositol 3-kinase/protein kinase B signal transduction",
  "gene_name": "Hematopoietic cell signal transducer",
  "gene_symbol": "HCST",
  "term_id": "GO:0051897"
}